{
  "term_label": "postsynapse",
  "term_id": "GO:0098794",
  "gene_name": "Gamma-aminobutyric acid receptor subunit alpha-3",
  "gene": "UniProtKB:P34903",
  "gene_symbol": "GABRA3"
}